{
  "gene": "UniProtKB:Q9NZD8",
  "gene_name": "Maspardin",
  "term_id": "GO:0042609",
  "gene_symbol": "SPG21",
  "term_label": "CD4 receptor binding"
}